{
  "gene_symbol": "PATE2",
  "term_label": "extracellular space",
  "term_id": "GO:0005615",
  "gene_name": "Prostate and testis expressed protein 2",
  "gene": "UniProtKB:Q6UY27"
}